{
  "gene_name": "SH2B adapter protein 2",
  "gene": "UniProtKB:O14492",
  "term_label": "B cell receptor signaling pathway",
  "gene_symbol": "SH2B2",
  "term_id": "GO:0050853"
}